{
  "gene": "UniProtKB:Q06330",
  "term_label": "MAML1-RBP-Jkappa- ICN1 complex",
  "gene_symbol": "RBPJ",
  "gene_name": "Recombining binding protein suppressor of hairless",
  "term_id": "GO:0002193"
}